{
  "gene_name": "Probable ATP-dependent RNA helicase DDX60-like",
  "term_id": "GO:0003725",
  "term_label": "double-stranded RNA binding",
  "gene_symbol": "DDX60L",
  "gene": "UniProtKB:Q5H9U9"
}